{
  "gene_name": "Syntaxin-7",
  "term_id": "GO:0005484",
  "term_label": "SNAP receptor activity",
  "gene_symbol": "STX7",
  "gene": "UniProtKB:O15400"
}